regulation of citrulline biosynthetic process [GO:1903248] (biological process) Subtypes: negative regulation of citrulline biosynthetic process [GO:1903249], positive regulation of citrulline biosynthetic process [GO:1903250] Also known as: regulation of citrulline anabolism, regulation of citrulline biosynthesis, regulation of citrulline formation, regulation of citrulline synthesis References: PMID:19278978 Sources: GOC:BHF, GOC:TermGenie, GOC:rl, GO_REF:0000058 Relationships: is a type of regulation of small molecule metabolic process [GO:0062012]; is a type of GO:2000282; regulates GO:0019240 Definition: Any process that modulates the frequency, rate or extent of citrulline biosynthetic process.